{
  "term_label": "regulation of mitochondrion organization",
  "gene": "UniProtKB:O00408",
  "term_id": "GO:0010821",
  "gene_name": "cGMP-dependent 3',5'-cyclic phosphodiesterase",
  "gene_symbol": "PDE2A"
}